intermembrane sterol transfer [GO:0120011] (biological process) References: PMID:20823909, PMID:24220498, PMID:25797198 Sources: GOC:krc Definition: The transport of sterols between membranes in which a sterol molecule is transported through an aqueous phase from the outer leaflet of a donor membrane to the outer leaflet of an acceptor membrane. This process does not require metabolic energy and can be either spontaneous or mediated by lipid transfer proteins (LTPs). Relationships: is a type of sterol transport [GO:0015918]; is a type of intermembrane lipid transfer [GO:0120009]